interleukin-32 production [GO:0072637] (biological process) Definition: The appearance of interleukin-32 due to biosynthesis or secretion following a cellular stimulus, resulting in an increase in its intracellular or extracellular levels. Regulation: regulated by regulation of interleukin-32 production [GO:0150189]; negatively regulated by negative regulation of interleukin-32 production [GO:0150190]; positively regulated by positive regulation of interleukin-32 production [GO:0150191] References: PMID:23729669 Sources: GOC:BHF, GOC:mah Relationships: is_a GO:0001816 Also known as: IL-32 production, IL32 production, NK4 production, TAIF production, interleukin-32 biosynthetic process, interleukin-32 secretion